{
  "gene_symbol": "LRPPRC",
  "gene_name": "Leucine-rich PPR motif-containing protein, mitochondrial",
  "gene": "UniProtKB:P42704",
  "term_id": "GO:0005739",
  "term_label": "mitochondrion"
}